{
  "term_label": "nucleus",
  "gene_symbol": "GPBP1",
  "gene": "UniProtKB:Q86WP2",
  "term_id": "GO:0005634",
  "gene_name": "Vasculin"
}